{
  "term_label": "structural constituent of ribosome",
  "gene": "UniProtKB:P82673",
  "gene_name": "Small ribosomal subunit protein mS35",
  "gene_symbol": "MRPS35",
  "term_id": "GO:0003735"
}